{
  "term_id": "UNKNOWN:0003",
  "gene_name": "Regulator of G-protein signaling 10",
  "gene": "UniProtKB:O43665",
  "gene_symbol": "RGS10",
  "term_label": "Unknown cellular component"
}